RNA-directed RNA polymerase complex [GO:0031379] (cellular component) Definition: A protein complex that possesses RNA-directed RNA polymerase activity. Sources: GOC:mah Relationships: is a type of GO:0030880 Subtypes: nuclear RNA-directed RNA polymerase complex [GO:0031380], viral RNA-directed RNA polymerase complex [GO:0031381], TERT-RMRP complex [GO:1990572]